{
  "term_label": "Unknown molecular function",
  "term_id": "UNKNOWN:0001",
  "gene_name": "Uncharacterized protein C6orf226",
  "gene": "UniProtKB:Q5I0X4",
  "gene_symbol": "C6orf226"
}